{
  "gene": "UniProtKB:O43679",
  "term_id": "GO:0045944",
  "gene_name": "LIM domain-binding protein 2",
  "gene_symbol": "LDB2",
  "term_label": "positive regulation of transcription by RNA polymerase II"
}